{
  "gene_symbol": "ANAPC16",
  "gene_name": "Anaphase-promoting complex subunit 16",
  "term_label": "Unknown molecular function",
  "term_id": "UNKNOWN:0001",
  "gene": "UniProtKB:Q96DE5"
}